{
  "gene_symbol": "ZDHHC19",
  "term_label": "protein-cysteine S-palmitoyltransferase activity",
  "gene": "UniProtKB:Q8WVZ1",
  "term_id": "GO:0019706",
  "gene_name": "Palmitoyltransferase ZDHHC19"
}